{
  "term_label": "intracellular zinc ion homeostasis",
  "gene_name": "Metallothionein-1B",
  "gene": "UniProtKB:P07438",
  "term_id": "GO:0006882",
  "gene_symbol": "MT1B"
}